{
  "term_label": "extracellular matrix structural constituent conferring tensile strength",
  "gene_name": "Collagen alpha-3(IV) chain",
  "gene": "UniProtKB:Q01955",
  "term_id": "GO:0030020",
  "gene_symbol": "COL4A3"
}